negative regulation of male germ-line stem cell asymmetric division [GO:1904839] (biological process) References: PMID:19339709 Sources: GOC:TermGenie, GO_REF:0000058 Relationships: is a type of negative regulation of cell development [GO:0010721]; is a type of GO:0045769; is a type of negative regulation of multicellular organismal process [GO:0051241]; is a type of regulation of male germ-line stem cell asymmetric division [GO:1904838]; negatively regulates male germ-line stem cell asymmetric division [GO:0048133] Definition: Any process that stops, prevents or reduces the frequency, rate or extent of male germ-line stem cell asymmetric division. Also known as: down regulation of male germ-line stem cell asymmetric division, down regulation of male germ-line stem cell renewal, down-regulation of male germ-line stem cell asymmetric division, down-regulation of male germ-line stem cell renewal, downregulation of male germ-line stem cell asymmetric division, downregulation of male germ-line stem cell renewal, negative regulation of male germ-line stem cell renewal, inhibition of male germ-line stem cell asymmetric division, inhibition of male germ-line stem cell renewal